{
  "gene_symbol": "TTC12",
  "gene_name": "Tetratricopeptide repeat protein 12",
  "term_label": "cytoplasm",
  "gene": "UniProtKB:Q9H892",
  "term_id": "GO:0005737"
}